{
  "gene_name": "Kinesin-like protein KIF21B",
  "gene": "UniProtKB:O75037",
  "gene_symbol": "KIF21B",
  "term_id": "GO:0016887",
  "term_label": "ATP hydrolysis activity"
}